{
  "gene_name": "Putative uncharacterized protein COL25A1-DT",
  "term_label": "Unknown cellular component",
  "gene_symbol": "COL25A1-DT",
  "term_id": "UNKNOWN:0003",
  "gene": "UniProtKB:Q6ZST2"
}